GBD domain binding [GO:0032427] (molecular function) References: PMID:9119069 Sources: GOC:mah, GOC:pg Definition: Binding to a GTPase protein binding domain (GDB) domain. The GBD is a short motif, including a minimum region of 16 amino acids, identified in proteins that bind to small GTPases such as Cdc42 and Rac. Also known as: CRIB motif binding, Cdc42/Rac interactive binding motif binding, P21-Rho-binding domain binding, PMD binding Relationships: is a type of GO:0019904